Gram-negative-bacterium-type cell outer membrane assembly [GO:0043165] (biological process) Sources: GOC:jl, ISBN:0135712254 Relationships: is a type of GO:0071709; is part of cell envelope organization [GO:0043163] Also known as: cell outer membrane biogenesis Definition: The assembly of an outer membrane of the type formed in Gram-negative bacteria. This membrane is enriched in polysaccharide and protein, and the outer leaflet of the membrane contains specific lipopolysaccharide structures.